response to fatty acid [GO:0070542] (biological process) Sources: GOC:lp Relationships: is a type of GO:0033993; is a type of GO:1901700 Definition: Any process that results in a change in state or activity of a cell or an organism (in terms of movement, secretion, enzyme production, gene expression, etc.) as a result of a fatty acid stimulus. Subtypes: response to jasmonic acid [GO:0009753], response to oleic acid [GO:0034201], GO:0070543, cellular response to fatty acid [GO:0071398], response to leptomycin B [GO:1901344], response to lipoic acid [GO:1903442], response to butyrate [GO:1903544], GO:1904550, response to ionomycin [GO:1904636], response to palmitoleic acid [GO:1904926], response to leukotriene B4 [GO:1905389]